{
  "term_id": "UNKNOWN:0003",
  "gene_symbol": "TDRD12",
  "gene_name": "Putative ATP-dependent RNA helicase TDRD12",
  "gene": "UniProtKB:Q587J7",
  "term_label": "Unknown cellular component"
}